{
  "term_label": "intermediate filament organization",
  "term_id": "GO:0045109",
  "gene_name": "Arf-GAP domain and FG repeat-containing protein 1",
  "gene_symbol": "AGFG1",
  "gene": "UniProtKB:P52594"
}